{
  "gene_symbol": "ITGB7",
  "term_label": "cell-cell adhesion",
  "gene": "UniProtKB:P26010",
  "gene_name": "Integrin beta-7",
  "term_id": "GO:0098609"
}